{
  "gene_name": "Catalase",
  "term_id": "GO:0005777",
  "gene_symbol": "CAT",
  "term_label": "peroxisome",
  "gene": "UniProtKB:P04040"
}